{
  "term_id": "GO:0034625",
  "gene_symbol": "ELOVL3",
  "term_label": "fatty acid elongation, monounsaturated fatty acid",
  "gene": "UniProtKB:Q9HB03",
  "gene_name": "Elongation of very long chain fatty acids protein 3"
}